{
  "term_id": "GO:0000978",
  "gene": "UniProtKB:Q9BUY5",
  "term_label": "RNA polymerase II cis-regulatory region sequence-specific DNA binding",
  "gene_name": "Zinc finger protein 426",
  "gene_symbol": "ZNF426"
}